{
  "gene_name": "DENN domain-containing protein 1A",
  "term_label": "endocytosis",
  "gene_symbol": "DENND1A",
  "term_id": "GO:0006897",
  "gene": "UniProtKB:Q8TEH3"
}